{
  "gene_name": "Stearoyl-CoA desaturase",
  "term_id": "GO:1903966",
  "gene_symbol": "SCD",
  "term_label": "monounsaturated fatty acid biosynthetic process",
  "gene": "UniProtKB:O00767"
}